{
  "gene_name": "Transmembrane protease serine 11B",
  "term_id": "GO:0005886",
  "gene": "UniProtKB:Q86T26",
  "gene_symbol": "TMPRSS11B",
  "term_label": "plasma membrane"
}